negative regulation of toll-like receptor 2 signaling pathway [GO:0034136] (biological process) Also known as: negative regulation of TLR2 signaling pathway, negative regulation of toll-like receptor 2 signalling pathway Relationships: is a type of negative regulation of immune system process [GO:0002683]; is a type of negative regulation of signal transduction [GO:0009968]; is a type of GO:0034135; negatively regulates toll-like receptor 2 signaling pathway [GO:0034134] References: PMID:16551253, PMID:17328678 Sources: GOC:add Definition: Any process that stops, prevents, or reduces the frequency, rate, or extent of toll-like receptor 2 signaling pathway.